seed dormancy process [GO:0010162] (biological process) Sources: GOC:PO_curators, GOC:lr, ISBN:9781405139830, PO_REF:00009 Definition: A dormancy process in which dormancy (sometimes called a dormant state) is induced, maintained or broken in a seed. Seed dormancy is a suspension of most physiological activity and growth in a seed, including the embryo contained therein, that can be reactivated. It often requires special conditions for reactivation, such as specific temperature, scarification, or leaching of inhibitors. Regulation: negatively regulated by negative regulation of seed dormancy process [GO:1902039]; positively regulated by positive regulation of seed dormancy process [GO:1902040]; RO_0002211 by regulation of seed dormancy process [GO:2000033] Relationships: is a type of developmental process involved in reproduction [GO:0003006]; is_a dormancy process [GO:0022611]; is a type of multicellular organismal process [GO:0032501]; is a type of GO:0048609; is part of seed maturation [GO:0010431] Subtypes: maintenance of seed dormancy [GO:0010231], GO:0048838 Also known as: seed dormancy